{
  "term_label": "ATPase-coupled intramembrane lipid transporter activity",
  "term_id": "GO:0140326",
  "gene_name": "Phospholipid-transporting ATPase IF",
  "gene_symbol": "ATP11B",
  "gene": "UniProtKB:Q9Y2G3"
}